ferritin receptor activity [GO:0070287] (molecular function) Definition: Combining with ferritin, and delivering ferritin into the cell via endocytosis. Relationships: is a type of cargo receptor activity [GO:0038024] References: PMID:17459943, PMID:19154717 Sources: GOC:bf Also known as: ferritin complex receptor activity